{
  "term_label": "extracellular space",
  "gene": "UniProtKB:P01036",
  "gene_symbol": "CST4",
  "term_id": "GO:0005615",
  "gene_name": "Cystatin-S"
}